biphenyl catabolic process [GO:0070980] (biological process) Also known as: biphenyl breakdown, biphenyl catabolism, biphenyl degradation Relationships: is a type of biphenyl metabolic process [GO:0018879]; is a type of xenobiotic catabolic process [GO:0042178] Definition: The chemical reactions and pathways resulting in the breakdown of biphenyl, a toxic aromatic hydrocarbon used as a heat transfer agent, as a fungistat in packaging citrus fruits and in plant disease control. Biphenyl can be chlorinated with 1-10 chlorine molecules to form polychlorinated biphenyls (PCBs). References: PMID:16310831, PMID:16339959